{
  "gene_name": "Probable fibrosin-1",
  "term_id": "UNKNOWN:0001",
  "gene_symbol": "FBRS",
  "term_label": "Unknown molecular function",
  "gene": "UniProtKB:Q9HAH7"
}